positive regulation of natural killer cell mediated immunity [GO:0002717] (biological process) Subtypes: positive regulation of natural killer cell cytokine production [GO:0002729], positive regulation of natural killer cell mediated immune response to tumor cell [GO:0002857], GO:0045954 Sources: GOC:add Also known as: positive regulation of NK cell mediated immunity, up regulation of natural killer cell mediated immunity, up-regulation of natural killer cell mediated immunity, upregulation of natural killer cell mediated immunity, activation of natural killer cell mediated immunity, stimulation of natural killer cell mediated immunity, positive regulation of NK cell activity, positive regulation of natural killer cell activity Definition: Any process that activates or increases the frequency, rate, or extent of natural killer cell mediated immunity. Relationships: is a type of positive regulation of lymphocyte mediated immunity [GO:0002708]; is a type of GO:0002715; is a type of GO:0045089; RO_0002213 natural killer cell mediated immunity [GO:0002228]